{
  "term_id": "UNKNOWN:0001",
  "term_label": "Unknown molecular function",
  "gene": "UniProtKB:A6NIK2",
  "gene_symbol": "LRRC10B",
  "gene_name": "Leucine-rich repeat-containing protein 10B"
}